{
  "term_label": "collagen type IX trimer",
  "gene": "UniProtKB:Q14050",
  "gene_name": "Collagen alpha-3(IX) chain",
  "term_id": "GO:0005594",
  "gene_symbol": "COL9A3"
}